{
  "term_label": "negative chemotaxis",
  "gene_symbol": "SEMA4D",
  "gene": "UniProtKB:Q92854",
  "gene_name": "Semaphorin-4D",
  "term_id": "GO:0050919"
}